{
  "term_id": "GO:0045944",
  "term_label": "positive regulation of transcription by RNA polymerase II",
  "gene_symbol": "SBNO2",
  "gene": "UniProtKB:Q9Y2G9",
  "gene_name": "Protein strawberry notch homolog 2"
}